{
  "gene_symbol": "ANXA9",
  "gene_name": "Annexin A9",
  "gene": "UniProtKB:O76027",
  "term_id": "GO:0005544",
  "term_label": "calcium-dependent phospholipid binding"
}